{
  "term_id": "GO:0004984",
  "gene_symbol": "OR13F1",
  "gene_name": "Olfactory receptor 13F1",
  "term_label": "olfactory receptor activity",
  "gene": "UniProtKB:Q8NGS4"
}